{
  "term_id": "GO:0032588",
  "gene": "UniProtKB:Q6ULP2",
  "gene_name": "Aftiphilin",
  "term_label": "trans-Golgi network membrane",
  "gene_symbol": "AFTPH"
}